{
  "gene_name": "PDZ domain-containing protein GIPC3",
  "gene": "UniProtKB:Q8TF64",
  "gene_symbol": "GIPC3",
  "term_id": "UNKNOWN:0002",
  "term_label": "Unknown biological process"
}